{
  "term_id": "GO:0030838",
  "gene_symbol": "CDC42EP2",
  "term_label": "positive regulation of actin filament polymerization",
  "gene_name": "Cdc42 effector protein 2",
  "gene": "UniProtKB:O14613"
}